{
  "gene_symbol": "CCL21",
  "gene_name": "C-C motif chemokine 21",
  "term_label": "positive regulation of cell migration",
  "term_id": "GO:0030335",
  "gene": "UniProtKB:O00585"
}